aerobic respiration, using ammonia as electron donor [GO:0019409] (biological process) Also known as: aerobic ammonia oxidation to nitrite via hydrazine, nitrification Sources: MetaCyc:AMMOXID-PWY Relationships: is a type of aerobic respiration [GO:0009060]; is a type of energy derivation by oxidation of reduced inorganic compounds [GO:0015975]; is a type of ammonia oxidation [GO:0019329]; is a type of nitrogen cycle metabolic process [GO:0071941] Definition: The metabolic process in which ammonia (NH3) is oxidized to nitrite (NO2) in the presence of oxygen; enzymatic reactions convert ammonia to hydrazine, and hydrazine to nitrite.